{
  "term_id": "GO:0004830",
  "gene_name": "Tryptophan--tRNA ligase, mitochondrial",
  "term_label": "tryptophan-tRNA ligase activity",
  "gene_symbol": "WARS2",
  "gene": "UniProtKB:Q9UGM6"
}